{
  "term_id": "GO:0000785",
  "gene_name": "T-box transcription factor TBX10",
  "gene": "UniProtKB:O75333",
  "term_label": "chromatin",
  "gene_symbol": "TBX10"
}